brain morphogenesis [GO:0048854] (biological process) Sources: GOC:dgh, GOC:jid Definition: The process in which the anatomical structures of the brain are generated and organized. The brain is one of the two components of the central nervous system and is the center of thought and emotion. It is responsible for the coordination and control of bodily activities and the interpretation of information from the senses (sight, hearing, smell, etc.). Relationships: is a type of GO:0009887; is part of brain development [GO:0007420]